spermidine synthase activity [GO:0004766] (molecular function) Also known as: S-adenosylmethioninamine:putrescine 3-aminopropyltransferase activity, SpeE, aminopropyltransferase activity, putrescine aminopropyltransferase activity, spermidine synthetase activity Relationships: is a type of transferase activity, transferring alkyl or aryl (other than methyl) groups [GO:0016765] Sources: EC:2.5.1.16 Definition: Catalysis of the reaction: S-adenosylmethioninamine + putrescine = 5'-methylthioadenosine + spermidine.